{
  "gene_symbol": "PTP4A3",
  "term_label": "nucleus",
  "gene_name": "Protein tyrosine phosphatase type IVA 3",
  "term_id": "GO:0005634",
  "gene": "UniProtKB:O75365"
}